{
  "gene_symbol": "HAS2",
  "term_id": "GO:0005886",
  "gene_name": "Hyaluronan synthase 2",
  "term_label": "plasma membrane",
  "gene": "UniProtKB:Q92819"
}